{
  "gene_symbol": "PTPRN",
  "term_id": "GO:0035773",
  "term_label": "insulin secretion involved in cellular response to glucose stimulus",
  "gene": "UniProtKB:Q16849",
  "gene_name": "Receptor-type tyrosine-protein phosphatase-like N"
}